axial mesoderm morphogenesis [GO:0048319] (biological process) Sources: GOC:go_curators Relationships: is a type of mesoderm morphogenesis [GO:0048332]; is part of axial mesoderm development [GO:0048318] Definition: The process in which the anatomical structures of the axial mesoderm are generated and organized.